positive regulation of adaptive immune memory response [GO:1905676] (biological process) Also known as: up regulation of adaptive immune memory response, up-regulation of adaptive immune memory response, upregulation of adaptive immune memory response, activation of adaptive immune memory response References: PMID:26831526 Sources: GOC:TermGenie, GO_REF:0000058 Relationships: is_a positive regulation of adaptive immune response [GO:0002821]; is a type of GO:1905674; positively regulates GO:0090716 Definition: Any process that activates or increases the frequency, rate or extent of adaptive immune memory response.